{
  "term_id": "GO:0032040",
  "term_label": "small-subunit processome",
  "gene_symbol": "NOL10",
  "gene_name": "Nucleolar protein 10",
  "gene": "UniProtKB:Q9BSC4"
}